{
  "gene_symbol": "TTC39C",
  "term_id": "UNKNOWN:0003",
  "gene": "UniProtKB:Q8N584",
  "gene_name": "Tetratricopeptide repeat protein 39C",
  "term_label": "Unknown cellular component"
}